{
  "term_label": "DNA-binding transcription factor activity, RNA polymerase II-specific",
  "gene_name": "Zinc finger protein 596",
  "gene_symbol": "ZNF596",
  "term_id": "GO:0000981",
  "gene": "UniProtKB:Q8TC21"
}